bromoxynil nitrilase activity [GO:0018761] (molecular function) Sources: RHEA:22100 Also known as: 3,5-dibromo-4-hydroxybenzonitrile aminohydrolase activity, bromoxynil-specific nitrilase activity Definition: Catalysis of the reaction: 3,5-dibromo-4-hydroxybenzonitrile + 2 H2O = 3,5-dibromo-4-hydroxybenzoate + NH4. Involved in the bacterial degradation of the herbicide bromoxynil. Relationships: is a type of nitrilase activity [GO:0000257]